cellular bud neck septin ring organization [GO:0032186] (BP) Definition: Control of the formation, spatial distribution, and breakdown of a septin ring located at the bud neck. Sources: GOC:mah Relationships: is a type of septin ring organization [GO:0031106]; is a type of mitotic cell cycle process [GO:1903047]; is part of mitotic cytokinesis [GO:0000281]; is part of cytokinesis, division site positioning [GO:0007105] Also known as: cellular bud neck septin ring organisation